{
  "gene_symbol": "WNT7B",
  "term_id": "GO:0060070",
  "gene": "UniProtKB:P56706",
  "gene_name": "Protein Wnt-7b",
  "term_label": "canonical Wnt signaling pathway"
}